indolylacetylinositol arabinosyltransferase activity [GO:0050409] (molecular function) Definition: Catalysis of the reaction: 1L-1-O-(indol-3-yl)acetyl-myo-inositol + UDP-L-arabinose = (indol-3-yl)acetyl-myo-inositol 3-L-arabinoside + H+ + UDP. Relationships: is a type of UDP-glycosyltransferase activity [GO:0008194]; is a type of arabinosyltransferase activity [GO:0052636] Sources: EC:2.4.2.34, RHEA:19505 Also known as: UDP-L-arabinose:(indol-3-yl)acetyl-myo-inositol L-arabinosyltransferase activity, UDP-L-arabinose:indol-3-ylacetyl-myo-inositol L-arabinosyltransferase activity, arabinosylindolylacetylinositol synthase activity